{
  "term_label": "peptide hormone binding",
  "gene_symbol": "SLC40A1",
  "term_id": "GO:0017046",
  "gene": "UniProtKB:Q9NP59",
  "gene_name": "Solute carrier family 40 member 1"
}